{
  "gene_symbol": "AVP",
  "gene": "UniProtKB:P01185",
  "gene_name": "Vasopressin-neurophysin 2-copeptin",
  "term_label": "neuropeptide hormone activity",
  "term_id": "GO:0005184"
}